{
  "gene": "UniProtKB:Q96RD7",
  "term_label": "plasma membrane",
  "gene_symbol": "PANX1",
  "gene_name": "Pannexin-1",
  "term_id": "GO:0005886"
}